light adaption [GO:0036367] (biological process) Definition: The ability of a photoreceptor to adjust to varying levels of light. Note: Light adaptation is usually a combination of cell desensitization and response acceleration. References: PMID:16039565 Sources: GOC:gap Relationships: is a type of response to light intensity [GO:0009642]